{
  "term_label": "defense response to bacterium",
  "gene": "UniProtKB:P05164",
  "gene_symbol": "MPO",
  "term_id": "GO:0042742",
  "gene_name": "Myeloperoxidase"
}